{
  "gene_symbol": "DLGAP4",
  "term_id": "GO:0060090",
  "term_label": "molecular adaptor activity",
  "gene_name": "Disks large-associated protein 4",
  "gene": "UniProtKB:Q9Y2H0"
}